{
  "term_label": "N-glycan processing",
  "gene_name": "Alpha-N-acetylneuraminide alpha-2,8-sialyltransferase",
  "gene": "UniProtKB:Q92185",
  "term_id": "GO:0006491",
  "gene_symbol": "ST8SIA1"
}